{
  "term_label": "immune response",
  "gene": "UniProtKB:P41597",
  "gene_symbol": "CCR2",
  "gene_name": "C-C chemokine receptor type 2",
  "term_id": "GO:0006955"
}